{
  "term_id": "GO:0042981",
  "gene": "UniProtKB:A6NCW0",
  "gene_symbol": "USP17L3",
  "gene_name": "Ubiquitin carboxyl-terminal hydrolase 17-like protein 3",
  "term_label": "regulation of apoptotic process"
}